{
  "term_label": "cellular response to calcium ion",
  "gene_name": "Copine-4",
  "gene_symbol": "CPNE4",
  "gene": "UniProtKB:Q96A23",
  "term_id": "GO:0071277"
}